{
  "gene_name": "Zinc finger protein 771",
  "gene_symbol": "ZNF771",
  "term_label": "DNA-binding transcription factor activity, RNA polymerase II-specific",
  "term_id": "GO:0000981",
  "gene": "UniProtKB:Q7L3S4"
}